negative regulation of hippocampal neuron apoptotic process [GO:0110091] (biological process) Relationships: is a type of negative regulation of neuron apoptotic process [GO:0043524]; is a type of regulation of hippocampal neuron apoptotic process [GO:0110089]; RO_0002212 GO:0110088 Definition: Any process that stops, prevents, or reduces the frequency, rate or extent of cell death by apoptotic process in hippocampal neurons. References: PMID:18940801 Sources: GOC:sl